regulation of blood coagulation, intrinsic pathway [GO:2000266] (biological process) Relationships: is a type of regulation of blood coagulation [GO:0030193]; is a type of regulation of protein activation cascade [GO:2000257]; regulates blood coagulation, intrinsic pathway [GO:0007597] Sources: GOC:mah Subtypes: negative regulation of blood coagulation, intrinsic pathway [GO:2000267], positive regulation of blood coagulation, intrinsic pathway [GO:2000268] Definition: Any process that modulates the frequency, rate or extent of blood coagulation, intrinsic pathway.